{
  "term_label": "positive regulation of proteasomal ubiquitin-dependent protein catabolic process",
  "gene": "UniProtKB:O15169",
  "term_id": "GO:0032436",
  "gene_name": "Axin-1",
  "gene_symbol": "AXIN1"
}